{
  "gene_symbol": "CABP4",
  "gene": "UniProtKB:P57796",
  "term_id": "GO:0007602",
  "gene_name": "Calcium-binding protein 4",
  "term_label": "phototransduction"
}